{
  "term_id": "GO:0032869",
  "term_label": "cellular response to insulin stimulus",
  "gene_name": "Phosphatidate phosphatase LPIN3",
  "gene_symbol": "LPIN3",
  "gene": "UniProtKB:Q9BQK8"
}